{
  "gene_symbol": "MMTAG2",
  "gene": "UniProtKB:Q9BU76",
  "term_label": "Unknown biological process",
  "gene_name": "Multiple myeloma tumor-associated protein 2",
  "term_id": "UNKNOWN:0002"
}